RNA helicase activity [GO:0003724] (molecular function) Also known as: ATP-dependent RNA helicase activity Definition: Unwinding of an RNA helix, driven by ATP hydrolysis. Regulation: regulated by regulation of RNA helicase activity [GO:1902280]; negatively regulated by RNA helicase inhibitor activity [GO:1990119] References: PMID:19158098 Sources: GOC:jl Relationships: is a type of helicase activity [GO:0004386]; is a type of GO:0008186; is_a catalytic activity, acting on RNA [GO:0140098] Subtypes: 5'-3' RNA helicase activity [GO:0032574], GO:0034458